{
  "term_id": "GO:0000242",
  "gene_symbol": "CDK5RAP2",
  "gene": "UniProtKB:Q96SN8",
  "gene_name": "CDK5 regulatory subunit-associated protein 2",
  "term_label": "pericentriolar material"
}